{
  "term_id": "UNKNOWN:0001",
  "gene_name": "Protein FAM47A",
  "gene_symbol": "FAM47A",
  "term_label": "Unknown molecular function",
  "gene": "UniProtKB:Q5JRC9"
}